{
  "gene_name": "Transmembrane protein 191B",
  "gene_symbol": "TMEM191B",
  "term_label": "Unknown cellular component",
  "term_id": "UNKNOWN:0003",
  "gene": "UniProtKB:P0C7N4"
}